alpha-amino acid metabolic process [GO:1901605] (biological process) Relationships: is a type of amino acid metabolic process [GO:0006520]; is_a carboxylic acid metabolic process [GO:0019752] Sources: GOC:TermGenie Subtypes: citrulline metabolic process [GO:0000052], alanine metabolic process [GO:0006522], arginine metabolic process [GO:0006525], aspartate metabolic process [GO:0006531], GO:0006534, glycine metabolic process [GO:0006544], isoleucine metabolic process [GO:0006549], lysine metabolic process [GO:0006553], methionine metabolic process [GO:0006555], valine metabolic process [GO:0006573], serotonin biosynthetic process from tryptophan [GO:0006587], ornithine metabolic process [GO:0006591], selenocysteine metabolic process [GO:0016259], 1-aminocyclopropane-1-carboxylate metabolic process [GO:0018871], nicotinate nucleotide biosynthetic process from tryptophan [GO:0019356], D-amino acid metabolic process [GO:0046416], homocysteine metabolic process [GO:0050667], GO:0070189, L-amino acid metabolic process [GO:0170033], sarcosine metabolic process [GO:1901052], alpha-amino acid catabolic process [GO:1901606], GO:1901607 Also known as: alpha-amino acid metabolism Definition: The chemical reactions and pathways involving an alpha-amino acid.